{
  "term_id": "GO:0000421",
  "gene": "UniProtKB:P13473",
  "term_label": "autophagosome membrane",
  "gene_symbol": "LAMP2",
  "gene_name": "Lysosome-associated membrane glycoprotein 2"
}